CH domain binding [GO:0051401] (molecular function) References: PMID:11911887 Sources: Prosite:PDOC50021 Definition: Binding to a calponin homology protein domain, a domain of 100 residues that occurs in signaling and cytoskeletal proteins. Also known as: calponin homology domain binding Relationships: is a type of protein domain specific binding [GO:0019904]